presynaptic modulation of chemical synaptic transmission [GO:0099171] (biological process) Definition: Any process, acting in the presynapse that results in modulation of chemical synaptic transmission. Subtypes: GO:0099161, regulation of protein catabolic process at presynapse, modulating synaptic transmission [GO:0099575], GO:0099577, induction of synaptic vesicle exocytosis by positive regulation of presynaptic cytosolic calcium ion concentration [GO:0099703] Sources: GOC:dos Relationships: is a type of GO:0050804; occurs in GO:0098793